spore wall [GO:0031160] (cellular component) Also known as: spore coat Definition: The specialized envelope lying outside the cell membrane of a spore. Relationships: is a type of GO:0005618 Subtypes: ascospore wall [GO:0005619], GO:0043591, sexual spore wall [GO:0097514], asexual spore wall [GO:0097515] Sources: GOC:mah, GOC:pg